{
  "gene_name": "Cholinesterase",
  "term_label": "choline metabolic process",
  "gene_symbol": "BCHE",
  "gene": "UniProtKB:P06276",
  "term_id": "GO:0019695"
}